{
  "term_label": "Golgi membrane",
  "term_id": "GO:0000139",
  "gene_symbol": "MAN1C1",
  "gene_name": "Mannosyl-oligosaccharide 1,2-alpha-mannosidase IC",
  "gene": "UniProtKB:Q9NR34"
}